{
  "term_id": "GO:0004693",
  "gene": "UniProtKB:Q9BWU1",
  "gene_name": "Cyclin-dependent kinase 19",
  "gene_symbol": "CDK19",
  "term_label": "cyclin-dependent protein serine/threonine kinase activity"
}